negative regulation of the force of heart contraction by acetylcholine [GO:0003060] (biological process) Relationships: is a type of negative regulation of the force of heart contraction by chemical signal [GO:0003108]; is part of regulation of systemic arterial blood pressure by acetylcholine [GO:0003068] Also known as: decreased force of heart contraction by acetylcholine Definition: The process in which acetylcholine released from vagus nerve endings binds to muscarinic receptors and decreases the force of heart muscle contraction. Sources: GOC:mtg_cardio, GOC:rl